{
  "term_label": "Unknown molecular function",
  "gene_name": "Transmembrane and coiled-coil domain protein 3",
  "term_id": "UNKNOWN:0001",
  "gene": "UniProtKB:Q9ULS5",
  "gene_symbol": "TMCC3"
}